snRNA methyltransferase activity [GO:0106346] (molecular function) Subtypes: U2 snRNA 2'-O-methyladenosine m6 methyltransferase activity [GO:0106347], U2 snRNA adenosine m6 methyltransferase activity [GO:0106348], U6 snRNA (adenine-(43)-N(6))-methyltransferase activity [GO:0120048], U6 snRNA (guanine-N(2))-methyltransferase activity [GO:0160230] References: PMID:27573892 Definition: Catalysis of the transfer of a methyl group from a donor to a nucleoside residue in an snRNA molecule. Relationships: is a type of GO:0008173